{
  "gene_symbol": "TSC1",
  "term_label": "regulation of cell cycle",
  "gene": "UniProtKB:Q92574",
  "gene_name": "Hamartin",
  "term_id": "GO:0051726"
}